{
  "gene_name": "NPC intracellular cholesterol transporter 1",
  "gene": "UniProtKB:O15118",
  "term_id": "GO:0005886",
  "term_label": "plasma membrane",
  "gene_symbol": "NPC1"
}